{
  "term_label": "Unknown molecular function",
  "gene_symbol": "FBXL4",
  "gene": "UniProtKB:Q9UKA2",
  "term_id": "UNKNOWN:0001",
  "gene_name": "F-box_LRR-repeat protein 4"
}